{
  "gene": "UniProtKB:O15360",
  "gene_name": "Fanconi anemia group A protein",
  "gene_symbol": "FANCA",
  "term_label": "regulation of regulatory T cell differentiation",
  "term_id": "GO:0045589"
}